temperature compensation of the circadian clock [GO:0010378] (biological process) Definition: The process in which the circadian clock maintains robust and accurate timing over a broad range of physiological temperatures. The circadian clock is an endogenous 24-h timer found in most eukaryotes and in photosynthetic bacteria. The clock drives rhythms in the physiology, biochemistry, and metabolism of the organisms. References: PMID:16617099 Relationships: is a type of response to temperature stimulus [GO:0009266]; is a type of regulation of circadian rhythm [GO:0042752] Also known as: regulation of the circadian clock by temperature